{
  "gene": "UniProtKB:Q8TDN7",
  "gene_name": "Alkaline ceramidase 1",
  "gene_symbol": "ACER1",
  "term_id": "GO:0005783",
  "term_label": "endoplasmic reticulum"
}